{
  "gene": "UniProtKB:P0CG31",
  "gene_symbol": "ZNF286B",
  "term_id": "GO:0005634",
  "gene_name": "Putative zinc finger protein 286B",
  "term_label": "nucleus"
}